{
  "gene": "UniProtKB:P55075",
  "gene_name": "Fibroblast growth factor 8",
  "gene_symbol": "FGF8",
  "term_id": "GO:0008284",
  "term_label": "positive regulation of cell population proliferation"
}